positive regulation of nitrosative stress-induced intrinsic apoptotic signaling pathway [GO:1905260] (biological process) Also known as: positive regulation of intrinsic apoptotic signaling pathway in response to nitrosative stress, up regulation of intrinsic apoptotic signaling pathway in response to nitrosative stress, up regulation of nitrosative stress-induced intrinsic apoptotic signaling pathway, up-regulation of intrinsic apoptotic signaling pathway in response to nitrosative stress, up-regulation of nitrosative stress-induced intrinsic apoptotic signaling pathway, upregulation of intrinsic apoptotic signaling pathway in response to nitrosative stress, upregulation of nitrosative stress-induced intrinsic apoptotic signaling pathway, activation of intrinsic apoptotic signaling pathway in response to nitrosative stress, activation of nitrosative stress-induced intrinsic apoptotic signaling pathway, activation of nitrosative stress-induced apoptosis, positive regulation of nitrosative stress-induced apoptosis, up regulation of nitrosative stress-induced apoptosis, up-regulation of nitrosative stress-induced apoptosis, upregulation of nitrosative stress-induced apoptosis Definition: Any process that activates or increases the frequency, rate or extent of intrinsic apoptotic signaling pathway in response to nitrosative stress. Sources: GOC:PARL, GOC:TermGenie, GOC:bf, GO_REF:0000058 Relationships: is a type of regulation of nitrosative stress-induced intrinsic apoptotic signaling pathway [GO:1905258]; is a type of GO:2001244; positively regulates intrinsic apoptotic signaling pathway in response to nitrosative stress [GO:1990442]